{
  "gene_name": "N-acetylneuraminate lyase",
  "term_id": "GO:0019262",
  "term_label": "N-acetylneuraminate catabolic process",
  "gene": "UniProtKB:Q9BXD5",
  "gene_symbol": "NPL"
}